cellular response to nocodazole [GO:1904403] (BP) Definition: Any process that results in a change in state or activity of a cell (in terms of movement, secretion, enzyme production, gene expression, etc.) as a result of a nocodazole stimulus. References: PMID:17822405 Sources: GOC:TermGenie, GO_REF:0000071 Relationships: is a type of GO:1901655; is a type of GO:1901699; is_a response to nocodazole [GO:1904402]